{
  "gene_name": "Tubulointerstitial nephritis antigen",
  "term_label": "Unknown biological process",
  "gene_symbol": "TINAG",
  "gene": "UniProtKB:Q9UJW2",
  "term_id": "UNKNOWN:0002"
}